{
  "term_label": "Notch signaling pathway",
  "term_id": "GO:0007219",
  "gene_symbol": "MIB1",
  "gene_name": "E3 ubiquitin-protein ligase MIB1",
  "gene": "UniProtKB:Q86YT6"
}